{
  "term_label": "early endosome",
  "gene_name": "Vacuolar protein sorting-associated protein 8 homolog",
  "term_id": "GO:0005769",
  "gene_symbol": "VPS8",
  "gene": "UniProtKB:Q8N3P4"
}